{
  "gene_symbol": "AXL",
  "gene_name": "Tyrosine-protein kinase receptor UFO",
  "gene": "UniProtKB:P30530",
  "term_id": "GO:0043066",
  "term_label": "negative regulation of apoptotic process"
}